{
  "gene": "UniProtKB:P50995",
  "term_id": "GO:0012506",
  "term_label": "vesicle membrane",
  "gene_symbol": "ANXA11",
  "gene_name": "Annexin A11"
}